{
  "gene_name": "Dynein axonemal heavy chain 3",
  "gene": "UniProtKB:Q8TD57",
  "term_label": "dynein intermediate chain binding",
  "gene_symbol": "DNAH3",
  "term_id": "GO:0045505"
}